pipecolic acid N-hydroxylase [GO:0062047] (molecular function) Definition: Catalysis of the reaction: L-pipecolic acid + NAD(P)H + O2 + H+ = N-hydroxypipecolic acid + NAD(P)+ + H2O. References: PMID:27758894, PMID:28330936 Relationships: is a type of GO:0016712